{
  "gene_symbol": "OC90",
  "gene": "UniProtKB:Q02509",
  "term_label": "calcium-dependent phospholipase A2 activity",
  "gene_name": "Otoconin-90",
  "term_id": "GO:0047498"
}